{
  "term_label": "Unknown cellular component",
  "gene_name": "Lipase member K",
  "gene": "UniProtKB:Q5VXJ0",
  "gene_symbol": "LIPK",
  "term_id": "UNKNOWN:0003"
}